negative regulation of presynapse assembly [GO:1905607] (biological process) Also known as: down regulation of presynapse assembly, down regulation of presynapse biogenesis, down regulation of presynaptic terminal assembly, down-regulation of presynapse assembly, down-regulation of presynapse biogenesis, down-regulation of presynaptic terminal assembly, downregulation of presynapse assembly, downregulation of presynapse biogenesis, downregulation of presynaptic terminal assembly, negative regulation of presynapse biogenesis, negative regulation of presynaptic terminal assembly, inhibition of presynapse assembly, inhibition of presynapse biogenesis, inhibition of presynaptic terminal assembly References: PMID:25533483 Sources: GOC:PARL, GOC:TermGenie, GOC:bc, GO_REF:0000058 Relationships: is a type of negative regulation of synapse assembly [GO:0051964]; is a type of regulation of presynapse assembly [GO:1905606]; negatively regulates presynapse assembly [GO:0099054] Subtypes: negative regulation of presynaptic active zone assembly [GO:1905519] Definition: Any process that stops, prevents or reduces the frequency, rate or extent of presynapse assembly.